{
  "gene_name": "Rabenosyn-5",
  "gene_symbol": "RBSN",
  "term_label": "Unknown molecular function",
  "term_id": "UNKNOWN:0001",
  "gene": "UniProtKB:Q9H1K0"
}